{
  "gene": "UniProtKB:O95271",
  "gene_name": "Poly [ADP-ribose] polymerase tankyrase-1",
  "term_label": "cytoplasm",
  "gene_symbol": "TNKS",
  "term_id": "GO:0005737"
}